negative regulation of artery smooth muscle contraction [GO:1905655] (biological process) References: PMID:27389411 Sources: GOC:BHF, GOC:BHF_miRNA, GOC:TermGenie, GOC:rph, GO_REF:0000058 Relationships: is a type of negative regulation of vascular associated smooth muscle contraction [GO:1904694]; is a type of regulation of artery smooth muscle contraction [GO:1905654]; negatively regulates artery smooth muscle contraction [GO:0014824] Also known as: down regulation of artery smooth muscle contraction, down-regulation of artery smooth muscle contraction, downregulation of artery smooth muscle contraction, inhibition of artery smooth muscle contraction Definition: Any process that stops, prevents or reduces the frequency, rate or extent of artery smooth muscle contraction.